posterior lateral line neuromast deposition [GO:0048922] (biological process) Definition: The process in which a migrating neuromast primordium deposits clusters of undifferentiated cells (proneuromasts) along its migratory path in the developing posterior lateral line. References: PMID:15832385 Relationships: is a type of neuromast deposition [GO:0048885]; BFO_0000050 GO:0048919